{
  "term_label": "malate metabolic process",
  "gene": "UniProtKB:P07954",
  "gene_name": "Fumarate hydratase, mitochondrial",
  "gene_symbol": "FH",
  "term_id": "GO:0006108"
}